{
  "gene_symbol": "ANKIB1",
  "term_label": "ubiquitin-dependent protein catabolic process",
  "gene": "UniProtKB:Q9P2G1",
  "term_id": "GO:0006511",
  "gene_name": "Ankyrin repeat and IBR domain-containing protein 1"
}